{
  "term_id": "GO:0005802",
  "gene_symbol": "YIPF7",
  "gene": "UniProtKB:Q8N8F6",
  "gene_name": "Protein YIPF7",
  "term_label": "trans-Golgi network"
}